{
  "gene_symbol": "SPDYE9",
  "term_id": "UNKNOWN:0002",
  "gene": "UniProtKB:A0A494C191",
  "term_label": "Unknown biological process",
  "gene_name": "Putative speedy protein E9"
}